{
  "gene": "UniProtKB:Q8N859",
  "term_label": "regulation of DNA-templated transcription",
  "gene_symbol": "ZNF713",
  "gene_name": "Zinc finger protein 713",
  "term_id": "GO:0006355"
}